multicellular organismal reproductive process [GO:0048609] (biological process) Relationships: is a type of reproductive process [GO:0022414] Definition: The process, occurring above the cellular level, that is pertinent to the reproductive function of a multicellular organism. This includes the integrated processes at the level of tissues and organs. Also known as: organismal reproductive process, reproductive process in a multicellular organism Sources: GOC:dph, GOC:jid, GOC:tb Subtypes: gamete generation [GO:0007276], insemination [GO:0007320], penetration of zona pellucida [GO:0007341], GO:0009900, seed dormancy process [GO:0010162], GO:0010431, GO:0019098, cellular process involved in reproduction in multicellular organism [GO:0022412], mammalian oogenesis stage [GO:0022605], ovulation [GO:0030728], genital disc sexually dimorphic development [GO:0035263], ovulation cycle [GO:0042698], sperm ejaculation [GO:0042713], penile erection [GO:0043084], sperm competition [GO:0046692], GO:0048624, maternal process involved in female pregnancy [GO:0060135], GO:0060136, maternal process involved in parturition [GO:0060137], fetal process involved in parturition [GO:0060138], GO:0060378, penetration of cumulus oophorus [GO:0061956], seminal clot liquefaction [GO:0070684], mucilage extrusion from seed coat [GO:0080001], GO:0160027, seed dehydration [GO:1990068]